{
  "gene_name": "CMT1A duplicated region transcript 15 protein-like protein",
  "gene": "UniProtKB:A8MXV6",
  "term_label": "Unknown cellular component",
  "term_id": "UNKNOWN:0003",
  "gene_symbol": "CDRT15L2"
}